{
  "gene_symbol": "CES2",
  "term_id": "GO:0050253",
  "gene": "UniProtKB:O00748",
  "gene_name": "Cocaine esterase",
  "term_label": "retinyl-palmitate esterase activity"
}